{
  "gene_name": "KATNB1-like protein 1",
  "term_label": "nucleolus",
  "gene": "UniProtKB:Q9H079",
  "gene_symbol": "KATNBL1",
  "term_id": "GO:0005730"
}